growth cone leading edge [GO:0061850] (cellular component) References: PMID:10797548 Subtypes: leading edge of axonal growth cone [GO:0061916], leading edge of dendritic growth cone [GO:0061917] Definition: That part of the growth cone which represents the distal part of the structure. Relationships: is a type of cell leading edge [GO:0031252]; is part of peripheral region of growth cone [GO:0090725]